{
  "term_id": "GO:0032153",
  "gene": "UniProtKB:Q99719",
  "gene_name": "Septin-5",
  "gene_symbol": "SEPTIN5",
  "term_label": "cell division site"
}